protein localization to cortical microtubule cytoskeleton [GO:0072699] (BP) Sources: GOC:mah Subtypes: protein localization to horsetail-astral microtubule array [GO:1903696] Relationships: is a type of protein localization to cell cortex [GO:0072697]; is a type of protein localization to microtubule cytoskeleton [GO:0072698] Definition: A process in which a protein is transported to, or maintained at, a location within the cortical microtubule cytoskeleton. Also known as: protein localisation to cortical microtubule cytoskeleton